{
  "term_id": "GO:0008017",
  "gene": "UniProtKB:Q6NUK4",
  "term_label": "microtubule binding",
  "gene_symbol": "REEP3",
  "gene_name": "Receptor expression-enhancing protein 3"
}